{
  "gene_symbol": "ALK",
  "term_id": "GO:0007169",
  "gene_name": "ALK tyrosine kinase receptor",
  "gene": "UniProtKB:Q9UM73",
  "term_label": "cell surface receptor protein tyrosine kinase signaling pathway"
}